{
  "gene_symbol": "NPM3",
  "gene_name": "Nucleoplasmin-3",
  "gene": "UniProtKB:O75607",
  "term_id": "GO:0005730",
  "term_label": "nucleolus"
}